{
  "term_id": "UNKNOWN:0003",
  "gene": "UniProtKB:Q6UXC1",
  "term_label": "Unknown cellular component",
  "gene_symbol": "MAMDC4",
  "gene_name": "Apical endosomal glycoprotein"
}